neuroinflammatory response [GO:0150076] (biological process) Regulation: regulated by regulation of neuroinflammatory response [GO:0150077]; positively regulated by positive regulation of neuroinflammatory response [GO:0150078]; negatively regulated by negative regulation of neuroinflammatory response [GO:0150079] Relationships: is a type of inflammatory response [GO:0006954] Definition: The immediate defensive reaction by neural vertebrate tissue to infection or injury caused by chemical or physical agents. Subtypes: reactive gliosis [GO:0150103] References: PMID:10981966, PMID:11099416, PMID:18164423 Sources: GOC:aruk, GOC:bc Also known as: nerve tissue inflammatory response, nervous tissue inflammatory response, neural tissue inflammatory response